eukaryotic translation initiation factor 3 complex [GO:0005852] (CC) References: PMID:15904532 Definition: A complex of several polypeptides that plays at least two important roles in protein synthesis: First, eIF3 binds to the 40S ribosome and facilitates loading of the Met-tRNA/eIF2.GTP ternary complex to form the 43S preinitiation complex. Subsequently, eIF3 apparently assists eIF4 in recruiting mRNAs to the 43S complex. The eIF3 complex contains five conserved core subunits, and may contain several additional proteins; the non-core subunits are thought to mediate association of the complex with specific sets of mRNAs. Relationships: is a type of protein-containing complex [GO:0032991]; is part of cytoplasm [GO:0005737] Subtypes: eukaryotic translation initiation factor 3 complex, eIF3e [GO:0071540], eukaryotic translation initiation factor 3 complex, eIF3m [GO:0071541] Also known as: eIF-3, eIF3